{
  "gene_symbol": "PRAMEF7",
  "gene_name": "PRAME family member 7",
  "gene": "UniProtKB:Q5VXH5",
  "term_label": "cytoplasm",
  "term_id": "GO:0005737"
}